{
  "gene": "UniProtKB:P49746",
  "gene_name": "Thrombospondin-3",
  "term_id": "GO:0031012",
  "term_label": "extracellular matrix",
  "gene_symbol": "THBS3"
}